{
  "term_id": "UNKNOWN:0001",
  "term_label": "Unknown molecular function",
  "gene_symbol": "MTMR12",
  "gene_name": "Myotubularin-related protein 12",
  "gene": "UniProtKB:Q9C0I1"
}